blood vessel endothelial cell fate commitment [GO:0060846] (biological process) Subtypes: GO:0060844, GO:0060845 Sources: GOC:dph, GOC:sdb_2009, GOC:tb Definition: The commitment of a cell to a blood vessel endothelial cell fate and its capacity to differentiate into a blood vessel endothelial cell. Relationships: is a type of endothelial cell fate commitment [GO:0060839]; is part of blood vessel endothelial cell differentiation [GO:0060837]